{
  "term_id": "UNKNOWN:0001",
  "term_label": "Unknown molecular function",
  "gene": "UniProtKB:O60732",
  "gene_name": "Melanoma-associated antigen C1",
  "gene_symbol": "MAGEC1"
}